{
  "gene_symbol": "ZNF761",
  "term_id": "GO:0006357",
  "gene": "UniProtKB:Q86XN6",
  "term_label": "regulation of transcription by RNA polymerase II",
  "gene_name": "Zinc finger protein 761"
}